{
  "gene_name": "Serine protease FAM111B",
  "gene_symbol": "FAM111B",
  "term_label": "replication fork processing",
  "gene": "UniProtKB:Q6SJ93",
  "term_id": "GO:0031297"
}